{
  "gene": "UniProtKB:Q9BYP7",
  "term_label": "regulation of monoatomic cation transmembrane transport",
  "gene_name": "Serine_threonine-protein kinase WNK3",
  "term_id": "GO:1904062",
  "gene_symbol": "WNK3"
}